{
  "gene": "UniProtKB:P07108",
  "term_label": "fatty-acyl-CoA binding",
  "term_id": "GO:0000062",
  "gene_name": "Acyl-CoA-binding protein",
  "gene_symbol": "DBI"
}